negative regulation of skeletal muscle acetylcholine-gated channel clustering [GO:1904394] (BP) Also known as: down regulation of skeletal muscle AChR clustering, down regulation of skeletal muscle acetylcholine-gated channel clustering, down regulation of skeletal muscle nicotinic acetylcholine receptor clustering, down-regulation of skeletal muscle AChR clustering, down-regulation of skeletal muscle acetylcholine-gated channel clustering, down-regulation of skeletal muscle nicotinic acetylcholine receptor clustering, downregulation of skeletal muscle AChR clustering, downregulation of skeletal muscle acetylcholine-gated channel clustering, downregulation of skeletal muscle nicotinic acetylcholine receptor clustering, negative regulation of skeletal muscle AChR clustering, negative regulation of skeletal muscle nicotinic acetylcholine receptor clustering, inhibition of skeletal muscle AChR clustering, inhibition of skeletal muscle acetylcholine-gated channel clustering, inhibition of skeletal muscle nicotinic acetylcholine receptor clustering Relationships: is a type of negative regulation of receptor clustering [GO:1903910]; is a type of regulation of skeletal muscle acetylcholine-gated channel clustering [GO:1904393]; negatively regulates skeletal muscle acetylcholine-gated channel clustering [GO:0071340] References: PMID:7722643 Sources: GOC:TermGenie, GO_REF:0000058 Definition: Any process that stops, prevents or reduces the frequency, rate or extent of skeletal muscle acetylcholine-gated channel clustering.